{
  "gene_name": "Flavin reductase (NADPH)",
  "term_label": "Unknown cellular component",
  "term_id": "UNKNOWN:0003",
  "gene": "UniProtKB:P30043",
  "gene_symbol": "BLVRB"
}